{
  "term_id": "UNKNOWN:0003",
  "gene_name": "Lymphocyte antigen 6 complex locus protein G6f",
  "gene_symbol": "LY6G6F",
  "gene": "UniProtKB:Q5SQ64",
  "term_label": "Unknown cellular component"
}